{
  "term_label": "defense response to virus",
  "term_id": "GO:0051607",
  "gene_symbol": "TLR7",
  "gene_name": "Toll-like receptor 7",
  "gene": "UniProtKB:Q9NYK1"
}